{
  "term_id": "UNKNOWN:0002",
  "gene": "UniProtKB:Q8TAL5",
  "gene_symbol": "C9orf43",
  "term_label": "Unknown biological process",
  "gene_name": "Uncharacterized protein C9orf43"
}